{
  "term_label": "Unknown cellular component",
  "gene_name": "WD repeat-containing protein 48",
  "term_id": "UNKNOWN:0003",
  "gene": "UniProtKB:Q8TAF3",
  "gene_symbol": "WDR48"
}